{
  "term_label": "plasma membrane",
  "gene_name": "Aquaporin-4",
  "term_id": "GO:0005886",
  "gene_symbol": "AQP4",
  "gene": "UniProtKB:P55087"
}